{
  "gene_symbol": "SNUPN",
  "gene": "UniProtKB:O95149",
  "term_label": "Unknown molecular function",
  "gene_name": "Snurportin-1",
  "term_id": "UNKNOWN:0001"
}